{
  "term_id": "UNKNOWN:0003",
  "gene_name": "von Willebrand factor A domain-containing protein 3B",
  "gene_symbol": "VWA3B",
  "term_label": "Unknown cellular component",
  "gene": "UniProtKB:Q502W6"
}